{
  "gene": "UniProtKB:Q562R1",
  "gene_name": "Beta-actin-like protein 2",
  "term_id": "GO:0098973",
  "term_label": "structural constituent of postsynaptic actin cytoskeleton",
  "gene_symbol": "ACTBL2"
}